ocellus pigment granule organization [GO:0008058] (biological process) Sources: http://fly.ebi.ac.uk/allied-data/lk/interactive-fly/aimain/1aahome.htm Relationships: is a type of pigment granule organization [GO:0048753] Also known as: ocellus pigment granule organisation, ocellus pigment granule organization and biogenesis Definition: A process that is carried out at the cellular level which results in the assembly, arrangement of constituent parts, or disassembly of intracellular pigment storage granules in the ocellus.